{
  "gene_symbol": "CCL23",
  "gene": "UniProtKB:P55773",
  "gene_name": "C-C motif chemokine 23",
  "term_label": "extracellular space",
  "term_id": "GO:0005615"
}